{
  "gene_symbol": "TPR",
  "term_label": "mRNA export from nucleus",
  "gene_name": "Nucleoprotein TPR",
  "term_id": "GO:0006406",
  "gene": "UniProtKB:P12270"
}